ceramide phosphoethanolamine catabolic process [GO:1905372] (biological process) Also known as: ceramide phosphoethanolamine breakdown, ceramide phosphoethanolamine catabolism, ceramide phosphoethanolamine degradation Definition: The chemical reactions and pathways resulting in the breakdown of ceramide phosphoethanolamine. References: PMID:25667419 Sources: GOC:TermGenie, GOC:hjd, GO_REF:0000068 Relationships: is a type of phospholipid catabolic process [GO:0009395]; is a type of GO:0030149